{
  "gene": "UniProtKB:Q8NGL3",
  "gene_name": "Olfactory receptor 5D14",
  "term_id": "GO:0004984",
  "gene_symbol": "OR5D14",
  "term_label": "olfactory receptor activity"
}